{
  "gene_name": "Stress-responsive DNAJB4-interacting membrane protein 1",
  "term_label": "Unknown biological process",
  "term_id": "UNKNOWN:0002",
  "gene": "UniProtKB:Q6ZPB5",
  "gene_symbol": "SDIM1"
}